{
  "gene": "UniProtKB:Q96TC7",
  "term_id": "UNKNOWN:0002",
  "gene_name": "Regulator of microtubule dynamics protein 3",
  "gene_symbol": "RMDN3",
  "term_label": "Unknown biological process"
}